{
  "gene": "UniProtKB:P68431",
  "gene_name": "Histone H3.1",
  "term_label": "nucleus",
  "gene_symbol": "H3C12",
  "term_id": "GO:0005634"
}